{
  "term_label": "calcium ion binding",
  "term_id": "GO:0005509",
  "gene_name": "Calbindin",
  "gene_symbol": "CALB1",
  "gene": "UniProtKB:P05937"
}